{
  "term_label": "membrane",
  "term_id": "GO:0016020",
  "gene": "UniProtKB:P59542",
  "gene_symbol": "TAS2R19",
  "gene_name": "Taste receptor type 2 member 19"
}